{
  "gene": "UniProtKB:Q13761",
  "term_id": "GO:0001503",
  "gene_name": "Runt-related transcription factor 3",
  "gene_symbol": "RUNX3",
  "term_label": "ossification"
}